{
  "gene_name": "Protein phosphatase 1M",
  "term_label": "mitochondrion",
  "term_id": "GO:0005739",
  "gene": "UniProtKB:Q96MI6",
  "gene_symbol": "PPM1M"
}